{
  "gene_name": "Aftiphilin",
  "gene_symbol": "AFTPH",
  "term_id": "GO:0030276",
  "term_label": "clathrin binding",
  "gene": "UniProtKB:Q6ULP2"
}